{
  "gene_name": "ADP_ATP translocase 1",
  "gene": "UniProtKB:P12235",
  "term_id": "GO:1990544",
  "gene_symbol": "SLC25A4",
  "term_label": "mitochondrial ATP transmembrane transport"
}